{
  "gene_symbol": "LCN15",
  "term_id": "UNKNOWN:0001",
  "term_label": "Unknown molecular function",
  "gene_name": "Lipocalin-15",
  "gene": "UniProtKB:Q6UWW0"
}